{
  "term_label": "phosphatidate phosphatase activity",
  "gene": "UniProtKB:Q9BQK8",
  "gene_name": "Phosphatidate phosphatase LPIN3",
  "gene_symbol": "LPIN3",
  "term_id": "GO:0008195"
}